cellular response to dopamine [GO:1903351] (biological process) Definition: Any process that results in a change in state or activity of a cell (in terms of movement, secretion, enzyme production, gene expression, etc.) as a result of a dopamine stimulus. References: PMID:11118945 Sources: GOC:TermGenie, GOC:mr, GO_REF:0000071 Relationships: is a type of cellular response to catecholamine stimulus [GO:0071870]; is_a response to dopamine [GO:1903350]